{
  "term_id": "GO:0007218",
  "term_label": "neuropeptide signaling pathway",
  "gene_name": "Neuropeptide Y receptor type 4-2",
  "gene_symbol": "NPY4R2",
  "gene": "UniProtKB:P0DQD5"
}